{
  "term_label": "melanosome organization",
  "term_id": "GO:0032438",
  "gene_name": "Ras-related protein Rab-32",
  "gene": "UniProtKB:Q13637",
  "gene_symbol": "RAB32"
}